{
  "gene_symbol": "SDHC",
  "term_label": "Unknown molecular function",
  "gene_name": "Succinate dehydrogenase cytochrome b560 subunit, mitochondrial",
  "term_id": "UNKNOWN:0001",
  "gene": "UniProtKB:Q99643"
}